axonal transport of mitochondrion [GO:0019896] (biological process) Sources: GOC:ai Subtypes: GO:0098957, retrograde axonal transport of mitochondrion [GO:0098958] Relationships: is a type of mitochondrion transport along microtubule [GO:0047497]; is a type of GO:0098930; occurs in axon cytoplasm [GO:1904115] Definition: The directed movement of mitochondria along microtubules in nerve cell axons. Also known as: axon transport of mitochondria